{
  "term_label": "intracellular sodium ion homeostasis",
  "gene": "UniProtKB:P50993",
  "gene_name": "Sodium_potassium-transporting ATPase subunit alpha-2",
  "gene_symbol": "ATP1A2",
  "term_id": "GO:0006883"
}